positive regulation of CD8-positive, alpha-beta T cell differentiation [GO:0043378] (biological process) Sources: GOC:add, ISBN:0781735149 Also known as: positive regulation of CD8-positive T lymphocyte differentiation, positive regulation of CD8-positive T-cell differentiation, positive regulation of CD8-positive T-lymphocyte differentiation, positive regulation of CD8-positive, alpha beta T lymphocyte differentiation, positive regulation of CD8-positive, alpha beta T-cell differentiation, positive regulation of CD8-positive, alpha beta T-lymphocyte differentiation, up regulation of CD8-positive, alpha-beta T cell differentiation, up-regulation of CD8-positive, alpha-beta T cell differentiation, upregulation of CD8-positive, alpha-beta T cell differentiation, activation of CD8-positive, alpha-beta T cell differentiation, stimulation of CD8-positive, alpha-beta T cell differentiation, positive regulation of CD8-positive, alpha-beta T cell development Relationships: is a type of regulation of CD8-positive, alpha-beta T cell differentiation [GO:0043376]; is a type of positive regulation of alpha-beta T cell differentiation [GO:0046638]; is a type of positive regulation of CD8-positive, alpha-beta T cell activation [GO:2001187]; positively regulates CD8-positive, alpha-beta T cell differentiation [GO:0043374] Definition: Any process that activates or increases the frequency, rate or extent of CD8-positive, alpha-beta T cell differentiation. Note: Note that immunologists typically use the word 'development' to refer to cells of B or T cell lineages undergoing the process that GO describes as 'cell differentiation'.